{
  "term_label": "Unknown molecular function",
  "gene": "UniProtKB:Q9BYE3",
  "term_id": "UNKNOWN:0001",
  "gene_symbol": "LCE3D",
  "gene_name": "Late cornified envelope protein 3D"
}